intracellular immature spore [GO:0042763] (CC) Relationships: is a type of GO:0110165 Subtypes: GO:0042601, ascospore-type prospore [GO:0042764] Definition: A cell or part of the cell that constitutes an early developmental stage of a spore, a small reproductive body that is highly resistant to desiccation and heat and is capable of growing into a new organism, produced especially by certain bacteria, fungi, algae, and nonflowering plants. Also known as: forespore Sources: GOC:jl, ISBN:0395825172